allantoate transport [GO:0015719] (biological process) Relationships: is a type of monocarboxylic acid transport [GO:0015718]; is a type of amide transport [GO:0042886] Definition: The directed movement of allantoate into, out of or within a cell, or between cells, by means of some agent such as a transporter or pore. Also known as: allantoin/allantoate transport Sources: GOC:krc